{
  "term_label": "SCAR complex",
  "term_id": "GO:0031209",
  "gene_name": "ABI gene family member 3",
  "gene_symbol": "ABI3",
  "gene": "UniProtKB:Q9P2A4"
}